{
  "gene_name": "Short-wave-sensitive opsin 1",
  "term_label": "phototransduction",
  "gene_symbol": "OPN1SW",
  "term_id": "GO:0007602",
  "gene": "UniProtKB:P03999"
}